{
  "gene_name": "Aquaporin-7B",
  "gene": "UniProtKB:A0A075B734",
  "term_id": "GO:0005886",
  "gene_symbol": "AQP7B",
  "term_label": "plasma membrane"
}